{
  "gene_symbol": "ATP8B4",
  "term_id": "GO:0007030",
  "term_label": "Golgi organization",
  "gene": "UniProtKB:Q8TF62",
  "gene_name": "Probable phospholipid-transporting ATPase IM"
}